regulation of thyroid hormone generation [GO:2000609] (biological process) Sources: GOC:obol Relationships: is a type of GO:0032350; regulates thyroid hormone generation [GO:0006590] Definition: Any process that modulates the frequency, rate or extent of thyroid hormone generation. Subtypes: GO:2000610, positive regulation of thyroid hormone generation [GO:2000611]